{
  "gene_name": "Protein FAM151B",
  "term_label": "Unknown molecular function",
  "term_id": "UNKNOWN:0001",
  "gene": "UniProtKB:Q6UXP7",
  "gene_symbol": "FAM151B"
}